{
  "gene": "UniProtKB:Q8NGD3",
  "gene_symbol": "OR4K5",
  "term_id": "UNKNOWN:0003",
  "term_label": "Unknown cellular component",
  "gene_name": "Olfactory receptor 4K5"
}